{
  "gene": "UniProtKB:Q5JVG2",
  "gene_name": "Zinc finger protein 484",
  "gene_symbol": "ZNF484",
  "term_label": "transcription cis-regulatory region binding",
  "term_id": "GO:0000976"
}